{
  "term_label": "RNA polymerase II cis-regulatory region sequence-specific DNA binding",
  "gene_symbol": "KLF6",
  "gene": "UniProtKB:Q99612",
  "gene_name": "Krueppel-like factor 6",
  "term_id": "GO:0000978"
}